rhamnose binding [GO:0033296] (molecular function) Definition: Binding to the D- or L-enantiomer of rhamnose. Relationships: is a type of monosaccharide binding [GO:0048029] Sources: GOC:mah